{
  "gene": "UniProtKB:Q07890",
  "gene_name": "Son of sevenless homolog 2",
  "gene_symbol": "SOS2",
  "term_id": "GO:0005886",
  "term_label": "plasma membrane"
}